{
  "gene": "UniProtKB:Q14004",
  "gene_symbol": "CDK13",
  "term_id": "GO:0008024",
  "term_label": "cyclin/CDK positive transcription elongation factor complex",
  "gene_name": "Cyclin-dependent kinase 13"
}